{
  "term_label": "Unknown molecular function",
  "gene_symbol": "B9D1",
  "term_id": "UNKNOWN:0001",
  "gene": "UniProtKB:Q9UPM9",
  "gene_name": "B9 domain-containing protein 1"
}